{
  "gene": "UniProtKB:Q9NQA3",
  "term_label": "exocytosis",
  "gene_symbol": "WASH6P",
  "gene_name": "WAS protein family homolog 6",
  "term_id": "GO:0006887"
}